{
  "term_id": "GO:0050766",
  "gene_symbol": "SIRPB1",
  "gene_name": "Signal-regulatory protein beta-1",
  "gene": "UniProtKB:O00241",
  "term_label": "positive regulation of phagocytosis"
}